{
  "gene_name": "Solute carrier family 12 member 9",
  "term_id": "GO:0055075",
  "gene": "UniProtKB:Q9BXP2",
  "term_label": "potassium ion homeostasis",
  "gene_symbol": "SLC12A9"
}